negative regulation of response to calcium ion [GO:1905946] (biological process) References: PMID:11404397 Sources: GOC:TermGenie, GOC:aruk, GOC:bc, GO_REF:0000058 Also known as: down regulation of response to Ca2+ ion, down regulation of response to calcium ion, down-regulation of response to Ca2+ ion, down-regulation of response to calcium ion, downregulation of response to Ca2+ ion, downregulation of response to calcium ion, negative regulation of response to Ca2+ ion, inhibition of response to Ca2+ ion, inhibition of response to calcium ion Definition: Any process that stops, prevents or reduces the frequency, rate or extent of response to calcium ion. Relationships: is a type of negative regulation of response to stimulus [GO:0048585]; is a type of GO:1905945; negatively regulates GO:0051592